{
  "term_id": "GO:0000981",
  "gene": "UniProtKB:P17028",
  "gene_name": "Zinc finger protein 24",
  "term_label": "DNA-binding transcription factor activity, RNA polymerase II-specific",
  "gene_symbol": "ZNF24"
}